{
  "gene_symbol": "TBC1D3C",
  "gene": "UniProtKB:Q6IPX1",
  "term_id": "GO:0005096",
  "gene_name": "TBC1 domain family member 3C",
  "term_label": "GTPase activator activity"
}